{
  "gene_name": "Polyadenylate-binding protein 1-like",
  "term_id": "GO:0008266",
  "gene": "UniProtKB:Q4VXU2",
  "term_label": "poly(U) RNA binding",
  "gene_symbol": "PABPC1L"
}